{
  "gene_symbol": "HBG2",
  "term_id": "GO:0031838",
  "gene": "UniProtKB:P69892",
  "gene_name": "Hemoglobin subunit gamma-2",
  "term_label": "haptoglobin-hemoglobin complex"
}